{
  "gene_name": "Plakophilin-2",
  "gene_symbol": "PKP2",
  "term_id": "GO:0007507",
  "gene": "UniProtKB:Q99959",
  "term_label": "heart development"
}